tyramine N-methyltransferase activity [GO:0030738] (MF) Sources: EC:2.1.1.27, RHEA:14865 Also known as: DIB O-methyltransferase (3,5-diiodo-4-hydroxy-benzoic acid), S-adenosyl-L-methionine:tyramine N-methyltransferase activity, S-adenosyl-methionine:tyramine N-methyltransferase activity, tyramine methylpherase activity Definition: Catalysis of the reaction: S-adenosyl-L-methionine + tyramine = N-methyltyramine + S-adenosyl-L-homocysteine + H+. Relationships: is a type of GO:0008757